peptidyl-cystine sulfhydration [GO:0044525] (biological process) Definition: The modification of a peptidyl-cystine residue in a protein by the addition of sulfur, to form peptidyl-cysteine persulfide. Relationships: is a type of protein sulfhydration [GO:0044524] Sources: GOC:jl, GOC:jsg